regulation of binding of sperm to zona pellucida [GO:2000359] (biological process) Relationships: is a type of regulation of cellular process [GO:0050794]; RO_0002211 binding of sperm to zona pellucida [GO:0007339] Also known as: regulation of ZPG binding Subtypes: negative regulation of binding of sperm to zona pellucida [GO:2000360] Definition: Any process that modulates the frequency, rate or extent of binding of sperm to the zona pellucida. Sources: GOC:obol